{
  "term_id": "GO:0001917",
  "gene": "UniProtKB:Q9Y6N9",
  "gene_name": "Harmonin",
  "term_label": "photoreceptor inner segment",
  "gene_symbol": "USH1C"
}